HDEL sequence binding [GO:0045015] (molecular function) Definition: Binding to a HDEL sequence, the C terminus tetrapeptide sequence His-Asp-Glu-Leu found in proteins that are to be retained in the endoplasmic reticulum. Also known as: HDEL receptor activity References: PMID:1327759 Relationships: is a type of ER retention sequence binding [GO:0046923]